{
  "term_label": "mRNA binding",
  "gene": "UniProtKB:A0A0J9YY54",
  "gene_symbol": "TEX13D",
  "term_id": "GO:0003729",
  "gene_name": "Testis-expressed protein 13D"
}